{
  "gene": "UniProtKB:Q8NGL1",
  "gene_symbol": "OR5D18",
  "term_id": "GO:0005549",
  "term_label": "odorant binding",
  "gene_name": "Olfactory receptor 5D18"
}